{
  "gene_symbol": "COQ8A",
  "term_id": "UNKNOWN:0001",
  "term_label": "Unknown molecular function",
  "gene": "UniProtKB:Q8NI60",
  "gene_name": "Atypical kinase COQ8A, mitochondrial"
}